{
  "gene": "UniProtKB:Q9BWF2",
  "term_id": "GO:0061630",
  "gene_name": "E3 ubiquitin-protein ligase TRAIP",
  "gene_symbol": "TRAIP",
  "term_label": "ubiquitin protein ligase activity"
}